{
  "term_label": "protein kinase activity",
  "gene_name": "Mitotic checkpoint serine_threonine-protein kinase BUB1",
  "gene": "UniProtKB:O43683",
  "term_id": "GO:0004672",
  "gene_symbol": "BUB1"
}